{
  "term_label": "histone H3K36 methyltransferase activity",
  "gene": "UniProtKB:Q96L73",
  "gene_name": "Histone-lysine N-methyltransferase, H3 lysine-36 specific",
  "term_id": "GO:0046975",
  "gene_symbol": "NSD1"
}